{
  "gene_symbol": "TSPYL2",
  "gene": "UniProtKB:Q9H2G4",
  "gene_name": "Testis-specific Y-encoded-like protein 2",
  "term_id": "GO:0042393",
  "term_label": "histone binding"
}